{
  "gene": "UniProtKB:Q9UK80",
  "term_id": "UNKNOWN:0001",
  "gene_name": "Ubiquitin carboxyl-terminal hydrolase 21",
  "gene_symbol": "USP21",
  "term_label": "Unknown molecular function"
}